{
  "gene_name": "Eukaryotic translation initiation factor 3 subunit E",
  "term_label": "eukaryotic translation initiation factor 3 complex",
  "gene_symbol": "EIF3E",
  "term_id": "GO:0005852",
  "gene": "UniProtKB:P60228"
}